positive regulation of excitatory postsynaptic potential [GO:2000463] (BP) Also known as: positive regulation of excitatory post-synaptic membrane potential, positive regulation of EPSP Subtypes: positive regulation of mini excitatory postsynaptic potential [GO:0061885] Sources: GOC:BHF, GOC:bf Relationships: is a type of positive regulation of signal transduction [GO:0009967]; is a type of modulation of excitatory postsynaptic potential [GO:0098815]; positively regulates GO:0060079 Definition: Any process that enhances the establishment or increases the extent of the excitatory postsynaptic potential (EPSP) which is a temporary increase in postsynaptic potential due to the flow of positively charged ions into the postsynaptic cell. The flow of ions that causes an EPSP is an excitatory postsynaptic current (EPSC) and makes it easier for the neuron to fire an action potential.